{
  "gene": "UniProtKB:Q8TEW8",
  "term_label": "establishment or maintenance of epithelial cell apical/basal polarity",
  "gene_symbol": "PARD3B",
  "term_id": "GO:0045197",
  "gene_name": "Partitioning defective 3 homolog B"
}